{
  "gene_name": "Matrix metalloproteinase-23",
  "term_label": "metalloendopeptidase activity",
  "term_id": "GO:0004222",
  "gene_symbol": "MMP23B",
  "gene": "UniProtKB:O75900"
}